negative regulation of apoptotic process involved in morphogenesis [GO:1902338] (biological process) Definition: Any process that stops, prevents or reduces the frequency, rate or extent of apoptotic process involved in morphogenesis. References: PMID:12202035 Sources: GOC:TermGenie, GOC:sart Also known as: down regulation of apoptotic process involved in morphogenesis, down-regulation of apoptotic process involved in morphogenesis, downregulation of apoptotic process involved in morphogenesis, down regulation of apoptosis involved in morphogenesis, down-regulation of apoptosis involved in morphogenesis, downregulation of apoptosis involved in morphogenesis, inhibition of apoptosis involved in morphogenesis, inhibition of apoptotic process involved in morphogenesis, negative regulation of apoptosis involved in morphogenesis, down regulation of apoptosis involved in development, down regulation of morphogenetic apoptosis, down-regulation of apoptosis involved in development, down-regulation of morphogenetic apoptosis, downregulation of apoptosis involved in development, downregulation of morphogenetic apoptosis, inhibition of apoptosis involved in development, inhibition of morphogenetic apoptosis, negative regulation of apoptosis involved in development, negative regulation of morphogenetic apoptosis Relationships: is a type of regulation of apoptotic process involved in morphogenesis [GO:1902337]; is a type of negative regulation of apoptotic process involved in development [GO:1904746]; negatively regulates apoptotic process involved in morphogenesis [GO:0060561] Subtypes: negative regulation of mesenchymal cell apoptotic process involved in nephron morphogenesis [GO:0072040], negative regulation of apoptotic process involved in outflow tract morphogenesis [GO:1902257]